{
  "gene_name": "Ethylmalonyl-CoA decarboxylase",
  "gene": "UniProtKB:Q9NTX5",
  "term_label": "carboxy-lyase activity",
  "term_id": "GO:0016831",
  "gene_symbol": "ECHDC1"
}